regulation of conjugation with cellular fusion [GO:0031137] (BP) Sources: GOC:mah Relationships: is a type of regulation of reproductive process [GO:2000241]; regulates conjugation with cellular fusion [GO:0000747] Subtypes: negative regulation of conjugation with cellular fusion [GO:0031138], GO:0031139, regulation of signal transduction involved in conjugation with cellular fusion [GO:0060238], regulation of induction of conjugation upon nitrogen starvation [GO:0060905] Definition: Any process that modulates the rate or frequency of conjugation with cellular fusion.